{
  "gene_symbol": "AVPI1",
  "gene_name": "Arginine vasopressin-induced protein 1",
  "term_id": "UNKNOWN:0003",
  "gene": "UniProtKB:Q5T686",
  "term_label": "Unknown cellular component"
}